{
  "gene_name": "Leucine-rich repeat and IQ domain-containing protein 1",
  "gene_symbol": "LRRIQ1",
  "term_id": "UNKNOWN:0002",
  "term_label": "Unknown biological process",
  "gene": "UniProtKB:Q96JM4"
}